renal tubule morphogenesis [GO:0061333] (biological process) Relationships: is a type of GO:0060562; BFO_0000050 renal tubule development [GO:0061326] Sources: GOC:dph, GOC:mtg_kidney_jan10 Definition: The process in which the renal tubule is generated by specification of cell fate, through the maintenance of cell polarity, regulated cell proliferation and morphogenetic cell rearrangements, shape changes and growth. A renal tubule is a tube that filters, re-absorbs and secretes substances to rid an organism of waste and to play a role in fluid homeostasis. Subtypes: Malpighian tubule morphogenesis [GO:0007443], nephron tubule morphogenesis [GO:0072078]